ribonuclease IX activity [GO:0033896] (molecular function) Definition: Catalysis of the endonucleolytic cleavage of poly(U) or poly(C) to fragments terminated by 3'-hydroxy and 5'-phosphate groups. Sources: EC:3.1.26.10 Also known as: poly(U)- and poly(C)-specific endoribonuclease activity Relationships: is a type of GO:0016891